{
  "term_id": "GO:0097352",
  "gene_name": "Tectonin beta-propeller repeat-containing protein 1",
  "term_label": "autophagosome maturation",
  "gene": "UniProtKB:Q7Z6L1",
  "gene_symbol": "TECPR1"
}